magnesium ion binding [GO:0000287] (molecular function) Definition: Binding to a magnesium (Mg) ion. Relationships: is a type of metal ion binding [GO:0046872] Sources: GOC:ai Also known as: Mg binding, magnesium binding